cGMP transport [GO:0070731] (biological process) Definition: The directed movement of cyclic GMP (cGMP), into, out of or within a cell. Sources: GOC:mah, ISBN:0198506732 Also known as: cyclic GMP transport Relationships: is a type of guanine nucleotide transport [GO:0001408]; is_a organic anion transport [GO:0015711]; is a type of purine ribonucleotide transport [GO:0015868]; is a type of cyclic nucleotide transport [GO:0070729]